{
  "gene_name": "Beta-defensin 133",
  "gene_symbol": "DEFB133",
  "gene": "UniProtKB:Q30KQ1",
  "term_label": "defense response to bacterium",
  "term_id": "GO:0042742"
}